{
  "gene_name": "A-kinase anchor protein 3",
  "gene_symbol": "AKAP3",
  "term_id": "GO:0005737",
  "term_label": "cytoplasm",
  "gene": "UniProtKB:O75969"
}